{
  "gene_symbol": "PSME1",
  "term_id": "GO:0005737",
  "gene": "UniProtKB:Q06323",
  "term_label": "cytoplasm",
  "gene_name": "Proteasome activator complex subunit 1"
}